{
  "gene_name": "Fascin-2",
  "term_id": "GO:0016477",
  "gene": "UniProtKB:O14926",
  "gene_symbol": "FSCN2",
  "term_label": "cell migration"
}